{
  "term_id": "GO:0000978",
  "gene": "UniProtKB:Q16676",
  "term_label": "RNA polymerase II cis-regulatory region sequence-specific DNA binding",
  "gene_symbol": "FOXD1",
  "gene_name": "Forkhead box protein D1"
}